{
  "gene_name": "Immunoglobulin heavy variable 3-21",
  "term_label": "antigen binding",
  "gene_symbol": "IGHV3-21",
  "gene": "UniProtKB:A0A0B4J1V1",
  "term_id": "GO:0003823"
}